symbiont-mediated suppression of host cytoplasmic pattern recognition receptor signaling pathway via inhibition of IRF3 activity [GO:0039548] (biological process) Relationships: is a type of symbiont-mediated suppression of cytoplasmic pattern recognition receptor signaling pathway [GO:0039537] References: PMID:21632562 Definition: A process in which a symbiont interferes with, inhibits or disrupts a cytoplasmic pattern recognition receptor signaling pathway in a host organism by reducing the activity of host IRF3 (interferon regulatory factor-3). IRF3 is a transcription factor in the RIG-I/MDA-5 signaling pathway. Viral infection triggers phosphorylation of cytoplasmic IRF3, which allows IRF3 to form a homodimer, migrate to the nucleus, and activate transcription of IFN-alpha and IFN-beta genes. Note: This term is for annotation of symbiont proteins that counteract the host anti-microbial innate immune response. Also known as: suppression by virus of host viral-induced cytoplasmic pattern recognition receptor signaling pathway via inhibition of IRF3 activity, inhibition of IRF3-dependent antiviral response, inhibition of host IRF3 by virus, suppression by virus of host IRF3 activity, suppression by virus of host interferon regulatory factor 3